{
  "term_id": "GO:0005667",
  "gene": "UniProtKB:Q9H808",
  "term_label": "transcription regulator complex",
  "gene_symbol": "TLE6",
  "gene_name": "Transducin-like enhancer protein 6"
}